ventral spinal cord interneuron fate determination [GO:0060580] (biological process) Relationships: is a type of neuron fate determination [GO:0048664]; is a type of GO:0060582; is part of ventral spinal cord interneuron fate commitment [GO:0060579] Sources: GOC:dph Definition: The process in which a cell becomes capable of differentiating autonomously into a ventral spinal cord interneuron regardless of its environment; upon determination, the cell fate cannot be reversed. Ventral spinal cord interneurons are cells located in the ventral portion of the spinal cord that transmit signals between sensory and motor neurons and are required for reflexive responses.